{
  "gene_symbol": "CDH4",
  "gene": "UniProtKB:P55283",
  "term_label": "calcium-dependent cell-cell adhesion",
  "term_id": "GO:0016339",
  "gene_name": "Cadherin-4"
}